{
  "gene": "UniProtKB:Q96LB2",
  "term_id": "GO:0005886",
  "gene_name": "Mas-related G-protein coupled receptor member X1",
  "gene_symbol": "MRGPRX1",
  "term_label": "plasma membrane"
}